{
  "term_id": "GO:0016607",
  "gene_symbol": "SRSF12",
  "gene_name": "Serine_arginine-rich splicing factor 12",
  "term_label": "nuclear speck",
  "gene": "UniProtKB:Q8WXF0"
}